{
  "term_label": "extracellular space",
  "gene": "UniProtKB:Q9Y4K0",
  "gene_name": "Lysyl oxidase homolog 2",
  "term_id": "GO:0005615",
  "gene_symbol": "LOXL2"
}